voltage-gated calcium channel activity involved in cardiac muscle cell action potential [GO:0086007] (molecular function) Definition: Enables the transmembrane transfer of a calcium ion by a voltage-gated channel across the plasma membrane of a cardiac muscle cell that contributes to the depolarization phase of an action potential. A voltage-gated channel is a channel whose open state is dependent on the voltage across the membrane in which it is embedded. Sources: GOC:BHF, GOC:mtg_cardiac_conduct_nov11 Relationships: is_a GO:0005245; is part of membrane depolarization during cardiac muscle cell action potential [GO:0086012] Subtypes: GO:0086056, voltage-gated calcium channel activity involved in bundle of His cell action potential [GO:0086057], voltage-gated calcium channel activity involved in Purkinje myocyte cell action potential [GO:0086058], voltage-gated calcium channel activity involved SA node cell action potential [GO:0086059]